{
  "gene_symbol": "CEP72",
  "term_label": "centriolar satellite",
  "gene": "UniProtKB:Q9P209",
  "term_id": "GO:0034451",
  "gene_name": "Centrosomal protein of 72 kDa"
}